convergent extension involved in nephron morphogenesis [GO:0072045] (BP) Definition: The morphogenetic process in which the renal epithelium narrows along one axis and lengthens in a perpendicular axis that contributes to the shaping of a nephron. Relationships: is a type of convergent extension involved in organogenesis [GO:0060029]; BFO_0000050 nephron morphogenesis [GO:0072028] Sources: GOC:mtg_kidney_jan10 Subtypes: convergent extension involved in mesonephric nephron morphogenesis [GO:0061237], convergent extension involved in metanephric nephron morphogenesis [GO:0072279]